{
  "gene_name": "Protein SAAL1",
  "term_id": "GO:1901647",
  "term_label": "positive regulation of synoviocyte proliferation",
  "gene": "UniProtKB:Q96ER3",
  "gene_symbol": "SAAL1"
}